{
  "gene": "UniProtKB:P28324",
  "term_label": "regulation of transcription by RNA polymerase II",
  "gene_name": "ETS domain-containing protein Elk-4",
  "gene_symbol": "ELK4",
  "term_id": "GO:0006357"
}